{
  "gene": "UniProtKB:P41146",
  "gene_name": "Nociceptin receptor",
  "gene_symbol": "OPRL1",
  "term_id": "GO:0007218",
  "term_label": "neuropeptide signaling pathway"
}